{
  "gene_name": "Oxidized low-density lipoprotein receptor 1",
  "gene_symbol": "OLR1",
  "term_id": "GO:0043235",
  "gene": "UniProtKB:P78380",
  "term_label": "receptor complex"
}